{
  "gene": "UniProtKB:Q9BZJ3",
  "term_label": "proteolysis",
  "term_id": "GO:0006508",
  "gene_symbol": "TPSD1",
  "gene_name": "Tryptase delta"
}